{
  "gene_name": "Cyclin-dependent kinase 9",
  "term_label": "transcription elongation by RNA polymerase II",
  "gene_symbol": "CDK9",
  "term_id": "GO:0006368",
  "gene": "UniProtKB:P50750"
}